{
  "term_id": "GO:0031012",
  "gene_name": "A disintegrin and metalloproteinase with thrombospondin motifs 5",
  "gene_symbol": "ADAMTS5",
  "term_label": "extracellular matrix",
  "gene": "UniProtKB:Q9UNA0"
}